diacylglycerol-dependent serine/threonine kinase activity [GO:0004697] (molecular function) Definition: Catalysis of the reaction: ATP + a protein = ADP + a phosphoprotein. This reaction requires diacylglycerol. Sources: EC:2.7.11.13 Also known as: PKC activity, diacylglycerol-activated phospholipid-dependent PKC activity, diacylglycerol-activated phospholipid-dependent protein kinase C activity, protein kinase Cepsilon activity, ATP:protein phosphotransferase (diacylglycerol-dependent) activity, PKC, PKCalpha, PKCbeta, PKCdelta, PKCepsilon, PKCgamma, Pkc1p, STK24, cPKC, cPKCalpha, cPKCbeta, cPKCgamma, nPKC, nPKCdelta, nPKCepsilon, nPKCeta, nPKCtheta Relationships: is a type of protein serine/threonine kinase activity [GO:0004674] Subtypes: calcium,diacylglycerol-dependent serine/threonine kinase activity [GO:0004698], GO:0004699 Regulation: negatively regulated by protein kinase C inhibitor activity [GO:0008426]; regulated by regulation of protein kinase C activity [GO:1900019]; positively regulated by positive regulation of protein kinase C activity [GO:1900020]